{
  "gene": "UniProtKB:Q5SY16",
  "term_id": "GO:0051731",
  "term_label": "polynucleotide 5'-hydroxyl-kinase activity",
  "gene_name": "Polynucleotide 5'-hydroxyl-kinase NOL9",
  "gene_symbol": "NOL9"
}